{
  "gene_name": "Olfactory receptor 52Z1P",
  "gene_symbol": "OR52Z1P",
  "gene": "UniProtKB:P0C646",
  "term_label": "olfactory receptor activity",
  "term_id": "GO:0004984"
}